viral capsid, internal space [GO:0098061] (cellular component) Sources: GOC:bm Relationships: is a type of virion component [GO:0044423] Also known as: internal head protein Definition: The region of a virus contained within the capsid shell, and usually containing the viral genome and accessory proteins.